{
  "term_label": "cytoplasm",
  "gene_name": "E3 ubiquitin-protein ligase TRIM11",
  "term_id": "GO:0005737",
  "gene": "UniProtKB:Q96F44",
  "gene_symbol": "TRIM11"
}